{
  "term_label": "Unknown biological process",
  "gene_name": "Serine_threonine-protein phosphatase 4 regulatory subunit 1",
  "term_id": "UNKNOWN:0002",
  "gene_symbol": "PPP4R1",
  "gene": "UniProtKB:Q8TF05"
}